{
  "gene": "UniProtKB:Q96S42",
  "term_label": "nodal signaling pathway",
  "term_id": "GO:0038092",
  "gene_symbol": "NODAL",
  "gene_name": "Nodal homolog"
}